{
  "gene": "UniProtKB:Q8N3V7",
  "gene_name": "Synaptopodin",
  "term_label": "actin binding",
  "gene_symbol": "SYNPO",
  "term_id": "GO:0003779"
}